{
  "gene_symbol": "GLDN",
  "gene_name": "Gliomedin",
  "term_label": "extracellular space",
  "term_id": "GO:0005615",
  "gene": "UniProtKB:Q6ZMI3"
}